(2R)-2-hydroxycarboxylate dehydrogenase activity [GO:0140174] (molecular function) Definition: Catalysis of the activity: a (2R)-2-hydroxycarboxylate + FAD + H+ = a 2-oxocarboxylate + FADH2. References: PMID:37863926 Sources: RHEA:82511 Relationships: is a type of (2R)-oxo-acid reductase activity [GO:0033719]